regulation of formation of radial glial scaffolds [GO:0061924] (biological process) Relationships: is a type of regulation of cell morphogenesis [GO:0022604]; regulates formation of radial glial scaffolds [GO:0021943] References: PMID:22076441 Definition: Any process that modulates the frequency, rate or extent of the formation of radial glial scaffolds. The scaffolds are used as a substrate for the radial migration of cells. Also known as: regulation of radial glial scaffold formation, regulation of Bergmann fiber biosynthesis, regulation of Bergmann fiber formation Subtypes: GO:0061925, positive regulation of formation of radial glial scaffolds [GO:0061926]